{
  "term_id": "GO:0004862",
  "term_label": "cAMP-dependent protein kinase inhibitor activity",
  "gene_name": "cAMP-dependent protein kinase type I-beta regulatory subunit",
  "gene": "UniProtKB:P31321",
  "gene_symbol": "PRKAR1B"
}